metanephric nephron morphogenesis [GO:0072273] (biological process) Definition: The process in which the anatomical structures of the metanephric nephron are generated and organized. A metanephric nephron is the functional unit of the metanephros. Relationships: is a type of GO:0072028; is part of metanephros morphogenesis [GO:0003338]; is part of metanephric nephron development [GO:0072210] Sources: GOC:mtg_kidney_jan10